{
  "gene_symbol": "SLC6A20",
  "gene_name": "Sodium- and chloride-dependent transporter XTRP3",
  "term_label": "plasma membrane",
  "term_id": "GO:0005886",
  "gene": "UniProtKB:Q9NP91"
}